HLA-G specific inhibitory MHC class Ib receptor activity [GO:0062083] (molecular function) Relationships: is a type of inhibitory MHC class Ib receptor activity [GO:0062080] Sources: DOI:10.1002/9780470015902.a0024246 Definition: Combining with a MHC class Ib molecule of the HLA-G subclass to mediate signaling that inhibits activation of a lymphocyte.